beta-alanine:pyruvate transaminase activity [GO:0016223] (molecular function) Definition: Catalysis of the reaction: L-alanine + 2-oxopropanoate = pyruvate + beta-alanine. Sources: RHEA:14077 Also known as: beta-alanine-pyruvate aminotransferase activity, L-alanine:3-oxopropanoate aminotransferase activity, beta-alanine--pyruvate aminotransferase activity, beta-alanine-alpha-alanine transaminase activity, omega-amino acid--pyruvate aminotransferase activity Relationships: is a type of transaminase activity [GO:0008483]